{
  "term_id": "GO:0031122",
  "gene": "UniProtKB:Q96CW5",
  "gene_symbol": "TUBGCP3",
  "gene_name": "Gamma-tubulin complex component 3",
  "term_label": "cytoplasmic microtubule organization"
}